tRNA-queuosine(34) beta-mannosyltransferase activity [GO:0016438] (molecular function) Relationships: is a type of mannosyltransferase activity [GO:0000030]; is a type of catalytic activity, acting on a tRNA [GO:0140101] Also known as: tRNA-queuosine beta-mannosyltransferase activity, GDP-mannose:tRNAAsp-queuosine O-5''-beta-D-mannosyltransferase activity Definition: Catalysis of the reaction: GDP-alpha-D-mannose + queuosine34 in tRNA(Asp) = GDP + H+ + O-4''-alpha-D-mannosylqueuosine34 in tRNA(Asp). Sources: RHEA:12885